{
  "term_label": "Unknown cellular component",
  "gene_symbol": "ZNF697",
  "gene": "UniProtKB:Q5TEC3",
  "gene_name": "Zinc finger protein 697",
  "term_id": "UNKNOWN:0003"
}